superior olivary nucleus formation [GO:0021720] (BP) Definition: The process that gives rise to the superior olivary nucleus. This process pertains to the initial formation of a structure from unspecified parts. In mice, the superior olivary nucleus is a small cylindrical mass on the dorsal surface of the lateral part of the trapezoid body of the pons, and it is situated immediately above the inferior olivary nucleus. It receives projections from the cochlear nucleus and thus is involved in the perception of sound. Relationships: is a type of GO:0048646; is part of GO:0021584; is part of superior olivary nucleus morphogenesis [GO:0021719] Sources: GOC:cls, GOC:dgh, GOC:dph, GOC:jid, GO_REF:0000021